{
  "term_label": "Unknown cellular component",
  "gene_symbol": "ST7L",
  "gene_name": "Suppressor of tumorigenicity 7 protein-like",
  "term_id": "UNKNOWN:0003",
  "gene": "UniProtKB:Q8TDW4"
}